{
  "gene": "UniProtKB:Q02790",
  "gene_symbol": "FKBP4",
  "gene_name": "Peptidyl-prolyl cis-trans isomerase FKBP4",
  "term_id": "GO:0006457",
  "term_label": "protein folding"
}